{
  "term_id": "GO:0006357",
  "gene_symbol": "ZNF442",
  "gene_name": "Zinc finger protein 442",
  "term_label": "regulation of transcription by RNA polymerase II",
  "gene": "UniProtKB:Q9H7R0"
}